sensory perception of itch [GO:0160025] (biological process) Definition: A sensory perception which causes the desire or reflex to scratch. References: PMID:26015312, PMID:29723501, PMID:30734045 Sources: Wikipedia:Itch Also known as: pruritus Relationships: is a type of sensory perception [GO:0007600]